phospholipase C-activating angiotensin-activated signaling pathway [GO:0086097] (biological process) Sources: GOC:BHF, GOC:bf, GOC:mtg_cardiac_conduct_nov11 Definition: A phospholipase C-activating G protein-coupled receptor signaling pathway initiated by angiotensin binding to its receptor on the surface of a target cell, and ending with the regulation of a downstream cellular process, e.g. transcription. Subtypes: phospholipase C-activating angiotensin-activated signaling pathway involved in heart process [GO:0086099] Relationships: is a type of phospholipase C-activating G protein-coupled receptor signaling pathway [GO:0007200]; is a type of angiotensin-activated signaling pathway [GO:0038166] Also known as: Gq-coupled angiotensin receptor signaling pathway, PLC-activating angiotensin receptor signaling pathway, angiotensin-mediated signaling pathway via activation of phospholipase C, phospholipase C-activating angiotensin receptor signaling pathway, phospholipase C-activating angiotensin-mediated signaling pathway